emericellamide catabolic process [GO:1900556] (biological process) Sources: GOC:TermGenie, GOC:di Relationships: is a type of lipid catabolic process [GO:0016042]; is a type of depsipeptide catabolic process [GO:0050762]; is a type of GO:0072340; is a type of secondary metabolite catabolic process [GO:0090487]; is a type of lactone catabolic process [GO:1901335] Subtypes: GO:1900616 Definition: The chemical reactions and pathways resulting in the breakdown of emericellamide. Also known as: emericellamide breakdown, emericellamide catabolism, emericellamide degradation